{
  "term_id": "GO:0005516",
  "gene": "UniProtKB:Q9UPW8",
  "gene_name": "Protein unc-13 homolog A",
  "gene_symbol": "UNC13A",
  "term_label": "calmodulin binding"
}